{
  "gene_symbol": "LINC01600",
  "term_id": "UNKNOWN:0002",
  "term_label": "Unknown biological process",
  "gene": "UniProtKB:Q96MT4",
  "gene_name": "Uncharacterized protein encoded by LINC01600"
}